{
  "term_label": "thiamine pyrophosphate binding",
  "gene_name": "Transketolase-like protein 1",
  "gene": "UniProtKB:P51854",
  "term_id": "GO:0030976",
  "gene_symbol": "TKTL1"
}